regulation of DNA repair [GO:0006282] (biological process) Relationships: is_a GO:0051052; is a type of regulation of cellular response to stress [GO:0080135]; regulates GO:0006281 Sources: GOC:go_curators Subtypes: GO:0032423, negative regulation of DNA repair [GO:0045738], positive regulation of DNA repair [GO:0045739], regulation of single strand break repair [GO:1903516], regulation of base-excision repair [GO:1905051], regulation of double-strand break repair [GO:2000779], GO:2000819 Definition: Any process that modulates the frequency, rate or extent of DNA repair.